interleukin-22 binding [GO:0042017] (molecular function) Definition: Binding to interleukin-22. Also known as: IL-22 binding Relationships: is a type of GO:0019955 Sources: GOC:jl